{
  "gene_symbol": "ARSG",
  "term_id": "GO:0004065",
  "term_label": "arylsulfatase activity",
  "gene_name": "Arylsulfatase G",
  "gene": "UniProtKB:Q96EG1"
}